{
  "term_id": "UNKNOWN:0001",
  "term_label": "Unknown molecular function",
  "gene_symbol": "COX8A",
  "gene_name": "Cytochrome c oxidase subunit 8A, mitochondrial",
  "gene": "UniProtKB:P10176"
}